{
  "term_label": "Unknown biological process",
  "term_id": "UNKNOWN:0002",
  "gene_symbol": "TSC22D2",
  "gene_name": "TSC22 domain family protein 2",
  "gene": "UniProtKB:O75157"
}